{
  "gene": "UniProtKB:Q9UHB9",
  "gene_name": "Signal recognition particle subunit SRP68",
  "term_id": "GO:0006614",
  "term_label": "SRP-dependent cotranslational protein targeting to membrane",
  "gene_symbol": "SRP68"
}